{
  "term_id": "GO:0016616",
  "term_label": "oxidoreductase activity, acting on the CH-OH group of donors, NAD or NADP as acceptor",
  "gene_symbol": "HSD3B1",
  "gene_name": "3 beta-hydroxysteroid dehydrogenase_Delta 5--4-isomerase type 1",
  "gene": "UniProtKB:P14060"
}